positive regulation of DNA-templated DNA replication [GO:2000105] (biological process) Relationships: is a type of positive regulation of DNA replication [GO:0045740]; is a type of regulation of DNA-templated DNA replication [GO:0090329]; positively regulates DNA-templated DNA replication [GO:0006261] Also known as: positive regulation of DNA-dependent DNA replication Definition: Any process that activates or increases the frequency, rate or extent of DNA-templated DNA replication. Subtypes: positive regulation of nuclear cell cycle DNA replication [GO:0010571], positive regulation of DNA-templated DNA replication initiation [GO:0032298], positive regulation of DNA endoreduplication [GO:0032877], positive regulation of mitochondrial DNA replication [GO:0090297] Sources: GOC:mah